positive regulation of amino acid biosynthetic process [GO:2000284] (biological process) Relationships: is a type of positive regulation of biosynthetic process [GO:0009891]; is a type of positive regulation of amino acid metabolic process [GO:0045764]; is a type of regulation of amino acid biosynthetic process [GO:2000282]; positively regulates GO:0008652 Subtypes: positive regulation of L-glutamine biosynthetic process [GO:0062134], positive regulation of histidine biosynthetic process [GO:0120215], positive regulation of arginine biosynthetic process [GO:1900080], positive regulation of homoserine biosynthetic process [GO:1901712], positive regulation of L-dopa biosynthetic process [GO:1903197], positive regulation of citrulline biosynthetic process [GO:1903250], positive regulation of lysine biosynthetic process via alpha-aminoadipate and saccharopine [GO:2001196], GO:2001278 Sources: GOC:obol Also known as: positive regulation of amino acid anabolism, positive regulation of amino acid biosynthesis, positive regulation of amino acid formation, positive regulation of amino acid synthesis, positive regulation of cellular amino acid biosynthetic process Definition: Any process that activates or increases the frequency, rate or extent of cellular amino acid biosynthetic process.